positive regulation of proteolysis associated with antigen processing and presentation [GO:0002630] (biological process) Relationships: is a type of GO:0002585; is a type of regulation of proteolysis associated with antigen processing and presentation [GO:0002628]; is a type of positive regulation of protein catabolic process [GO:0045732]; is_a positive regulation of proteolysis involved in protein catabolic process [GO:1903052]; positively regulates GO:0002496 Definition: Any process that activates or increases the frequency, rate, or extent of proteolysis associated with antigen processing and presentation. Also known as: up regulation of proteolysis associated with antigen processing and presentation, up-regulation of proteolysis associated with antigen processing and presentation, upregulation of proteolysis associated with antigen processing and presentation, activation of proteolysis associated with antigen processing and presentation, stimulation of proteolysis associated with antigen processing and presentation Sources: GOC:add